{
  "term_label": "RNA polymerase II cis-regulatory region sequence-specific DNA binding",
  "gene_name": "Zinc finger and BTB domain-containing protein 12",
  "term_id": "GO:0000978",
  "gene": "UniProtKB:Q9Y330",
  "gene_symbol": "ZBTB12"
}